{
  "gene_symbol": "ESYT1",
  "term_id": "GO:0031210",
  "gene_name": "Extended synaptotagmin-1",
  "gene": "UniProtKB:Q9BSJ8",
  "term_label": "phosphatidylcholine binding"
}